{
  "gene_symbol": "HTR6",
  "gene": "UniProtKB:P50406",
  "term_id": "GO:0030425",
  "gene_name": "5-hydroxytryptamine receptor 6",
  "term_label": "dendrite"
}